{
  "gene_name": "D(1A) dopamine receptor",
  "gene_symbol": "DRD1",
  "term_label": "G protein-coupled dopamine receptor signaling pathway",
  "term_id": "GO:0007212",
  "gene": "UniProtKB:P21728"
}